{
  "gene_name": "Protein fem-1 homolog A",
  "term_label": "proteasome-mediated ubiquitin-dependent protein catabolic process",
  "gene": "UniProtKB:Q9BSK4",
  "term_id": "GO:0043161",
  "gene_symbol": "FEM1A"
}